{
  "gene_symbol": "APOL5",
  "term_label": "Unknown cellular component",
  "term_id": "UNKNOWN:0003",
  "gene_name": "Apolipoprotein L5",
  "gene": "UniProtKB:Q9BWW9"
}